{
  "term_id": "UNKNOWN:0003",
  "term_label": "Unknown cellular component",
  "gene": "UniProtKB:A0A1B0GTL2",
  "gene_symbol": "C20orf204",
  "gene_name": "Uncharacterized protein C20orf204"
}